{
  "term_label": "negative regulation of transcription by RNA polymerase II",
  "gene_symbol": "NR2F6",
  "term_id": "GO:0000122",
  "gene_name": "Nuclear receptor subfamily 2 group F member 6",
  "gene": "UniProtKB:P10588"
}